{
  "gene_symbol": "ABCA8",
  "gene_name": "ABC-type organic anion transporter ABCA8",
  "term_label": "Unknown cellular component",
  "term_id": "UNKNOWN:0003",
  "gene": "UniProtKB:O94911"
}